RNA polymerase II preinitiation complex assembly [GO:0051123] (biological process) Definition: The formation of a large multiprotein-DNA complex that self-assembles on gene promoter through the sequential recruitment of the general initiation factors that compose the preinitiation complex (PIC) (which may include TFIIA, TFIIB, TFIID, TFIIE, TFIIF, and TFIIH complexes). The PIC engages RNA polymerase II on its DNA template strand and sparks polymerization of the first few RNA nucleotides of the nascent transcript, of which 8 are base-paired with the DNA template within a DNA bubble. PIC assembly may result in a pause step, which marks the end of the PIC assembly and may be followed by promoter clearance (exact synonym: promoter escape). For RNA polymerase II PIC assembly is preceded by the formation of a nucleosome-free region that allows the transcription machinery to access the promoter DNA. Relationships: is a type of transcription preinitiation complex assembly [GO:0070897]; BFO_0000050 transcription initiation at RNA polymerase II promoter [GO:0006367] References: PMID:15020047, PMID:31300188 Sources: GOC:txnOH Also known as: RNA polymerase II transcription PIC biosynthesis, RNA polymerase II transcription PIC formation, RNA polymerase II transcriptional preinitiation complex assembly, RNA polymerase II transcriptional preinitiation complex formation Regulation: negatively regulated by negative regulation of RNA polymerase II transcription preinitiation complex assembly [GO:0017055]; regulated by regulation of RNA polymerase II transcription preinitiation complex assembly [GO:0045898]; positively regulated by positive regulation of RNA polymerase II transcription preinitiation complex assembly [GO:0045899]